{
  "term_id": "GO:0097730",
  "gene_symbol": "IFT88",
  "gene": "UniProtKB:Q13099",
  "gene_name": "Intraflagellar transport protein 88 homolog",
  "term_label": "non-motile cilium"
}